{
  "gene": "UniProtKB:Q8N3A8",
  "term_id": "GO:0016020",
  "gene_name": "Protein mono-ADP-ribosyltransferase PARP8",
  "term_label": "membrane",
  "gene_symbol": "PARP8"
}